{
  "gene_name": "Proteasome activator complex subunit 2",
  "term_id": "GO:0061136",
  "gene": "UniProtKB:Q9UL46",
  "term_label": "regulation of proteasomal protein catabolic process",
  "gene_symbol": "PSME2"
}